{
  "gene": "UniProtKB:Q03938",
  "gene_symbol": "ZNF90",
  "term_label": "RNA polymerase II cis-regulatory region sequence-specific DNA binding",
  "term_id": "GO:0000978",
  "gene_name": "Zinc finger protein 90"
}